{
  "gene_symbol": "GFRA3",
  "gene": "UniProtKB:O60609",
  "gene_name": "GDNF family receptor alpha-3",
  "term_label": "signaling receptor activity",
  "term_id": "GO:0038023"
}